{
  "gene_name": "Proton-coupled amino acid transporter 1",
  "gene_symbol": "SLC36A1",
  "term_label": "L-proline transmembrane transporter activity",
  "term_id": "GO:0015193",
  "gene": "UniProtKB:Q7Z2H8"
}